{
  "term_label": "CORVET complex",
  "gene_symbol": "VPS8",
  "gene_name": "Vacuolar protein sorting-associated protein 8 homolog",
  "gene": "UniProtKB:Q8N3P4",
  "term_id": "GO:0033263"
}